protein serine/threonine/tyrosine kinase activity [GO:0004712] (molecular function) Definition: Catalysis of the reactions: ATP + a protein serine = ADP + protein serine phosphate; ATP + a protein threonine = ADP + protein threonine phosphate; and ATP + a protein tyrosine = ADP + protein tyrosine phosphate. Relationships: is a type of protein kinase activity [GO:0004672] Sources: GOC:mah Subtypes: MAP kinase kinase activity [GO:0004708] Also known as: dual-specificity kinase activity, dual-specificity protein kinase, protein threonine/tyrosine kinase activity